positive regulation of cell fate determination [GO:1905935] (biological process) Also known as: up regulation of cell fate determination, up-regulation of cell fate determination, upregulation of cell fate determination, activation of cell fate determination Definition: Any process that activates or increases the frequency, rate or extent of cell fate determination. Relationships: is a type of positive regulation of cellular process [GO:0048522]; is a type of positive regulation of developmental process [GO:0051094]; is a type of GO:1905933; positively regulates GO:0001709 Subtypes: GO:0048336 References: PMID:25793578 Sources: GOC:TermGenie, GOC:bhm, GO_REF:0000058